{
  "gene_name": "Myosin-IIIa",
  "gene": "UniProtKB:Q8NEV4",
  "term_label": "protein serine/threonine kinase activity",
  "gene_symbol": "MYO3A",
  "term_id": "GO:0004674"
}